detection of light stimulus involved in magnetoreception [GO:0050980] (biological process) References: PMID:15886990 Sources: GOC:ai, GOC:dos, Wikipedia:Magnetoception Also known as: magnetoreception, detection of light stimulus, magnetoreception, sensory detection of light stimulus, magnetoreception, sensory transduction of light stimulus, sensory detection of light stimulus during magnetoreception, sensory transduction of light stimulus during magnetoreception Relationships: is a type of detection of light stimulus involved in sensory perception [GO:0050962]; BFO_0000050 magnetoreception [GO:0050958] Definition: The series of events involved in magnetoception in which a light stimulus is received and converted into a molecular signal. Downstream processing of the light information in addition to other sensory data allows organisms to perceive the orientation of a magnetic field.